mesonephric glomerular capillary formation [GO:0061249] (biological process) Relationships: is a type of glomerular capillary formation [GO:0072104]; is part of GO:0061248 Definition: The process that gives rise to a mesonephric glomerular capillary. This process pertains to the initial formation of a structure from unspecified parts. Sources: GOC:mtg_kidney_jan10